{
  "term_label": "DNA-binding transcription factor activity, RNA polymerase II-specific",
  "gene": "UniProtKB:O43680",
  "gene_name": "Transcription factor 21",
  "term_id": "GO:0000981",
  "gene_symbol": "TCF21"
}